{
  "gene_name": "Rieske domain-containing protein",
  "gene_symbol": "RFESD",
  "term_id": "GO:0051537",
  "term_label": "2 iron, 2 sulfur cluster binding",
  "gene": "UniProtKB:Q8TAC1"
}